{
  "gene": "UniProtKB:Q8N3F9",
  "gene_name": "Integral membrane protein GPR137C",
  "term_id": "UNKNOWN:0001",
  "gene_symbol": "GPR137C",
  "term_label": "Unknown molecular function"
}